{
  "gene_symbol": "FAT4",
  "term_label": "Unknown molecular function",
  "term_id": "UNKNOWN:0001",
  "gene_name": "Protocadherin Fat 4",
  "gene": "UniProtKB:Q6V0I7"
}